{
  "gene": "UniProtKB:Q8N6S5",
  "gene_symbol": "ARL6IP6",
  "term_id": "UNKNOWN:0001",
  "term_label": "Unknown molecular function",
  "gene_name": "ADP-ribosylation factor-like protein 6-interacting protein 6"
}